{
  "term_id": "GO:0005615",
  "term_label": "extracellular space",
  "gene_symbol": "MMP9",
  "gene": "UniProtKB:P14780",
  "gene_name": "Matrix metalloproteinase-9"
}